{
  "gene": "UniProtKB:Q96T55",
  "gene_name": "Potassium channel subfamily K member 16",
  "gene_symbol": "KCNK16",
  "term_id": "GO:0005886",
  "term_label": "plasma membrane"
}